female courtship behavior [GO:0008050] (biological process) Sources: GOC:bf, GOC:pr Definition: The behavior of a female, for the purpose of attracting a sexual partner. Relationships: is a type of courtship behavior [GO:0007619]; is a type of GO:0060180 Also known as: female courtship behaviour